{
  "gene_name": "Acyl-coenzyme A thioesterase 1",
  "gene_symbol": "ACOT1",
  "gene": "UniProtKB:Q86TX2",
  "term_label": "Unknown cellular component",
  "term_id": "UNKNOWN:0003"
}